{
  "term_label": "double-strand break repair via homologous recombination",
  "gene": "UniProtKB:Q14159",
  "gene_symbol": "SPIDR",
  "gene_name": "DNA repair-scaffolding protein",
  "term_id": "GO:0000724"
}